histone H3K14 deacetylase activity, NAD-dependent [GO:0032041] (molecular function) Relationships: is a type of histone deacetylase activity, NAD-dependent [GO:0017136]; is a type of histone H3K deacetylase activity [GO:0141050] Definition: Catalysis of the reaction: histone H3 N6-acetyl-L-lysine (position 14) + NAD+ + H2O = histone H3 L-lysine (position 14) + 2''-O-acetyl-ADP-D-ribose + nicotinamide. This reaction transfers an acetyl group attached to a lysine residue in H3K14 to NAD, producing nicotinamide. References: PMID:28450737 Also known as: NAD-dependent histone H3-K14 deacetylase activity, NAD-dependent histone H3K14 deacetylase activity, NAD-dependent histone deacetylase activity (H3-K14 specific) Note: Comment: Note that the residue position corresponds to the canonical human H3 histone (UniProtKB:P84243); this residue is conserved across all eukaryotes. Residue 1 is the first residue following removal of the initiating Methionine (Met). Note that each histone is encoded by multiple genes, and sequences may vary across different genes within an organism.